lamellocyte differentiation [GO:0035171] (biological process) Definition: The process in which a relatively unspecialized hemocyte precursor cell acquires the specialized features of a lamellocyte. Lamellocytes are a hemocyte lineage that exists only in larvae, but are seldom observed in healthy animals. Lamellocytes differentiate massively in the lymph glands after parasitization and are large flat cells devoted to encapsulation of invaders too large to be phagocytosed by plasmatocytes. Regulation: regulated by GO:0035203; RO_0002212 by negative regulation of lamellocyte differentiation [GO:0035204]; positively regulated by positive regulation of lamellocyte differentiation [GO:0035205] Relationships: is a type of larval lymph gland hemocyte differentiation [GO:0035168] Also known as: lamellocyte cell differentiation References: PMID:14734104 Sources: GOC:bf